{
  "term_label": "nucleus",
  "term_id": "GO:0005634",
  "gene_name": "Tau-tubulin kinase 2",
  "gene": "UniProtKB:Q6IQ55",
  "gene_symbol": "TTBK2"
}